{
  "term_id": "UNKNOWN:0001",
  "gene_name": "Cullin-associated NEDD8-dissociated protein 2",
  "gene": "UniProtKB:O75155",
  "term_label": "Unknown molecular function",
  "gene_symbol": "CAND2"
}